{
  "term_label": "calcium-dependent protein binding",
  "term_id": "GO:0048306",
  "gene_name": "Protein S100-A6",
  "gene_symbol": "S100A6",
  "gene": "UniProtKB:P06703"
}